{
  "term_label": "G protein-coupled receptor signaling pathway",
  "term_id": "GO:0007186",
  "gene": "UniProtKB:Q8N0Y5",
  "gene_name": "Olfactory receptor 8I2",
  "gene_symbol": "OR8I2"
}